{
  "gene": "UniProtKB:Q9HAT0",
  "term_label": "Unknown molecular function",
  "gene_symbol": "ROPN1",
  "term_id": "UNKNOWN:0001",
  "gene_name": "Ropporin-1A"
}